putrescine metabolic process [GO:0009445] (biological process) Also known as: putrescine metabolism Sources: GOC:ai Subtypes: putrescine biosynthetic process [GO:0009446], putrescine catabolic process [GO:0009447], putrescine acetylation [GO:0032920] Definition: The chemical reactions and pathways involving putrescine, 1,4-diaminobutane; putrescine can be formed by decarboxylation of ornithine and is the metabolic precursor of spermidine and spermine. Relationships: is a type of polyamine metabolic process [GO:0006595]